histone H1 acetyltransferase activity [GO:0160262] (molecular function) Definition: Catalysis of the reaction: acetyl-CoA + histone H1 = CoA + acetyl-histone H1. References: PMID:40240600 Relationships: is a type of histone acetyltransferase activity [GO:0004402] Subtypes: histone H1-4K34 acetyltransferase activity [GO:0140187], histone H1K75 acetyltransferase activity [GO:0160263]